{
  "term_label": "guanyl-nucleotide exchange factor activity",
  "gene": "UniProtKB:Q5JSP0",
  "gene_name": "FYVE, RhoGEF and PH domain-containing protein 3",
  "gene_symbol": "FGD3",
  "term_id": "GO:0005085"
}